thalianol hydroxylase activity [GO:0080014] (molecular function) References: PMID:17474751, PMID:18356490 Sources: MetaCyc:RXN-9631 Definition: Catalysis of the reaction: a thalianol = a thalian-diol. This reaction is the addition of a hydroxyl group to thalianol ((13R,14R,17E)-podioda-8,17,21-trien-3beta-ol) to create a thalian-diol ((13R,14R,17E)-podioda-8,17,21-trien-3beta,X-diol), where the hydroxyl group may be attached at one of several different available carbons in ring B or C of thalianol, indicated by the X. Relationships: is a type of oxidoreductase activity, acting on paired donors, with incorporation or reduction of molecular oxygen, reduced flavin or flavoprotein as one donor, and incorporation of one atom of oxygen [GO:0016712] Note: In Field and Osbourn 2008 (PMID:18356490), thalianol is referred to as (3S,13S,3R)-malabarica-8,17,21-trien-3-ol and thalian-diol is referred to as (3S,13S,14R)-malabarica-8,17,21-trien-3,?-diol, but the error in this naming system was pointed out in Kolesnikova 2007 (PMID:17474751). The new names used in the definition have been approved by the authors (Field and Osbourn 2008).